regulation of triglyceride storage [GO:0010889] (biological process) Subtypes: GO:0010890, negative regulation of triglyceride storage [GO:0010891] Definition: Any process that modulates the rate, frequency or extent of sequestering of triglyceride. Triglyceride sequestration is the process of binding or confining any triester of glycerol such that it is separated from other components of a biological system. Also known as: regulation of sequestering of triacylglycerol, regulation of sequestering of triglyceride, regulation of triacylglycerol sequestration Relationships: is a type of GO:0010883; regulates triglyceride storage [GO:0030730] Sources: GOC:BHF, GOC:dph, GOC:tb